{
  "term_id": "GO:0030036",
  "gene_symbol": "MICAL3",
  "gene": "UniProtKB:Q7RTP6",
  "term_label": "actin cytoskeleton organization",
  "gene_name": "[F-actin]-monooxygenase MICAL3"
}